{
  "term_id": "UNKNOWN:0001",
  "gene_name": "Leucine-rich repeat transmembrane protein FLRT3",
  "gene_symbol": "FLRT3",
  "term_label": "Unknown molecular function",
  "gene": "UniProtKB:Q9NZU0"
}